{
  "term_id": "UNKNOWN:0002",
  "gene_symbol": "SHISAL2A",
  "gene_name": "Protein shisa-like-2A",
  "gene": "UniProtKB:Q6UWV7",
  "term_label": "Unknown biological process"
}